pivalyl-CoA mutase activity [GO:0034784] (molecular function) Note: Pivalyl-CoA is a synonym for 2,2-dimethylpropanoyl-CoA. Definition: Catalysis of the reaction: 3-methylbutanoyl-CoA = 2,2-dimethylpropanoyl-CoA. Sources: RHEA:52620 Relationships: is a type of intramolecular transferase activity [GO:0016866]